PcG protein complex [GO:0031519] (cellular component) Definition: A chromatin-associated multiprotein complex containing Polycomb Group proteins. In Drosophila, Polycomb group proteins are involved in the long-term maintenance of gene repression, and PcG protein complexes associate with Polycomb group response elements (PREs) in target genes to regulate higher-order chromatin structure. Relationships: is a type of nuclear protein-containing complex [GO:0140513] Also known as: Polycomb Group protein complex Subtypes: ESC/E(Z) complex [GO:0035098], GO:0035102, PR-DUB complex [GO:0035517] References: PMID:9372908